{
  "term_label": "chloride transmembrane transport",
  "gene_symbol": "SLC26A8",
  "term_id": "GO:1902476",
  "gene_name": "Testis anion transporter 1",
  "gene": "UniProtKB:Q96RN1"
}